{
  "gene_name": "DNA repair protein XRCC1",
  "term_id": "GO:0005634",
  "gene": "UniProtKB:P18887",
  "term_label": "nucleus",
  "gene_symbol": "XRCC1"
}